complement-dependent cytotoxicity [GO:0097278] (BP) Relationships: is a type of cell killing [GO:0001906]; has part GO:0006956 Sources: GOC:add, GOC:rv Definition: Cell killing caused by the membrane attack complex formed following complement activation. Regulation: RO_0002211 by regulation of complement-dependent cytotoxicity [GO:1903659]; negatively regulated by negative regulation of complement-dependent cytotoxicity [GO:1903660]; positively regulated by positive regulation of complement-dependent cytotoxicity [GO:1903661]